{
  "gene_symbol": "IQCA1L",
  "gene_name": "IQ and AAA domain-containing protein 1-like",
  "term_id": "GO:0016887",
  "gene": "UniProtKB:A6NCM1",
  "term_label": "ATP hydrolysis activity"
}